{
  "term_label": "telomeric DNA binding",
  "gene": "UniProtKB:Q9NYB0",
  "gene_name": "Telomeric repeat-binding factor 2-interacting protein 1",
  "term_id": "GO:0042162",
  "gene_symbol": "TERF2IP"
}